inulin binding [GO:2001082] (molecular function) Sources: GOC:mengo_curators Relationships: is a type of GO:0030247 Definition: Binding to inulin.